{
  "gene": "UniProtKB:Q9Y3C6",
  "gene_name": "Peptidyl-prolyl cis-trans isomerase-like 1",
  "gene_symbol": "PPIL1",
  "term_id": "GO:0071013",
  "term_label": "catalytic step 2 spliceosome"
}